larval central nervous system remodeling [GO:0035193] (biological process) References: PMID:9647692 Sources: GOC:sensu Also known as: CNS metamorphosis, central nervous system metamorphosis, larval central nervous system remodelling Definition: Reorganization of the pre-existing, functional larval central nervous system into one that can serve the novel behavioral needs of the adult. An example of this process is found in Drosophila melanogaster. Relationships: is a type of post-embryonic animal morphogenesis [GO:0009886]; is part of instar larval or pupal development [GO:0002165]; is part of central nervous system development [GO:0007417]